{
  "gene_symbol": "RAD51C",
  "gene": "UniProtKB:O43502",
  "term_label": "Rad51B-Rad51C-Rad51D-XRCC2 complex",
  "term_id": "GO:0033063",
  "gene_name": "DNA repair protein RAD51 homolog 3"
}